{
  "gene_symbol": "NKAP",
  "gene": "UniProtKB:Q8N5F7",
  "term_label": "chromatin binding",
  "term_id": "GO:0003682",
  "gene_name": "NF-kappa-B-activating protein"
}